{
  "term_id": "GO:0006396",
  "gene_symbol": "DNTTIP2",
  "gene_name": "Deoxynucleotidyltransferase terminal-interacting protein 2",
  "term_label": "RNA processing",
  "gene": "UniProtKB:Q5QJE6"
}